{
  "term_label": "rRNA catabolic process",
  "term_id": "GO:0016075",
  "gene": "UniProtKB:Q9NQT4",
  "gene_name": "Exosome complex component RRP46",
  "gene_symbol": "EXOSC5"
}